{
  "gene": "UniProtKB:Q9P2E2",
  "term_id": "GO:0005737",
  "gene_name": "Kinesin-like protein KIF17",
  "term_label": "cytoplasm",
  "gene_symbol": "KIF17"
}